{
  "term_id": "GO:0060396",
  "gene_symbol": "GH2",
  "term_label": "growth hormone receptor signaling pathway",
  "gene_name": "Growth hormone variant",
  "gene": "UniProtKB:P01242"
}